{
  "gene": "UniProtKB:Q9P2D0",
  "term_label": "nucleoplasm",
  "gene_name": "Inhibitor of Bruton tyrosine kinase",
  "term_id": "GO:0005654",
  "gene_symbol": "IBTK"
}